{
  "gene_name": "Interferon alpha-16",
  "term_label": "type I interferon-mediated signaling pathway",
  "gene": "UniProtKB:P05015",
  "term_id": "GO:0060337",
  "gene_symbol": "IFNA16"
}